{
  "gene": "UniProtKB:Q12824",
  "gene_symbol": "SMARCB1",
  "term_id": "GO:0003713",
  "term_label": "transcription coactivator activity",
  "gene_name": "SWI_SNF-related matrix-associated actin-dependent regulator of chromatin subfamily B member 1"
}